viral budding [GO:0046755] (biological process) Sources: ISBN:0781718325, VZ:1947 Definition: A viral process by which enveloped viruses acquire a host-derived membrane enriched in viral proteins to form their external envelope. The process starts when nucleocapsids, assembled or in the process of being built, induce formation of a membrane curvature in the host plasma or organelle membrane and wrap up in the forming bud. The process ends when the bud is eventually pinched off by membrane scission to release the enveloped particle into the lumenal or extracellular space. Also known as: virion budding, viral capsid envelopment, virus budding Subtypes: viral budding via host ESCRT complex [GO:0039702], viral budding from Golgi membrane [GO:0046760], viral budding from plasma membrane [GO:0046761], viral budding from endoplasmic reticulum membrane [GO:0046762], viral budding from nuclear membrane [GO:0046765] Relationships: is a type of viral process [GO:0016032]; is part of virion assembly [GO:0019068]